{
  "term_label": "mitochondrial outer membrane",
  "term_id": "GO:0005741",
  "gene_name": "Translocator protein 2",
  "gene": "UniProtKB:Q5TGU0",
  "gene_symbol": "TSPO2"
}